{
  "term_label": "Unknown biological process",
  "gene": "UniProtKB:Q86SX6",
  "term_id": "UNKNOWN:0002",
  "gene_name": "Glutaredoxin-related protein 5, mitochondrial",
  "gene_symbol": "GLRX5"
}